{
  "term_label": "cell-cell junction",
  "gene": "UniProtKB:O60711",
  "gene_name": "Leupaxin",
  "term_id": "GO:0005911",
  "gene_symbol": "LPXN"
}